{
  "gene_symbol": "NFS1",
  "term_id": "GO:0005739",
  "gene_name": "Cysteine desulfurase",
  "term_label": "mitochondrion",
  "gene": "UniProtKB:Q9Y697"
}